molybdenum-iron nitrogenase complex [GO:0016612] (cellular component) Relationships: is a type of nitrogenase complex [GO:0016610] References: PMID:11566366 Definition: An enzyme complex containing a molybdenum-iron cluster found in many species. It is composed of two proteins, dinitrogenase and nitrogenase reductase; dinitrogenase, the molybdenum-iron protein, is tetrameric with an alpha2-beta2 structure, and nitrogenase reductase is a homodimer. Also known as: molybdenum-iron nitrogenase activity